PSI associated light-harvesting complex I [GO:0009518] (cellular component) Subtypes: PSI associated light-harvesting complex I, LHCIa subcomplex [GO:0030083], PSI associated light-harvesting complex I, LHCIb subcomplex [GO:0030084] Also known as: LHCI Definition: Protein-pigment complex associated with photosystem I. Sources: GOC:lr Relationships: is a type of thylakoid light-harvesting complex [GO:0009503]